microtubule anchoring at mitotic spindle pole body [GO:1990810] (BP) Relationships: is a type of microtubule anchoring at spindle pole body [GO:0034631]; is a type of microtubule cytoskeleton organization involved in mitosis [GO:1902850]; is part of mitotic spindle assembly [GO:0090307] References: PMID:17486116 Definition: Any process in which a microtubule is maintained in a specific location in a cell by attachment to a mitotic spindle pole body. Microtubules attach to spindle pole bodies at the minus end.